{
  "term_label": "ADP-ribosylglutamate hydrolase activity",
  "gene": "UniProtKB:Q9BQ69",
  "term_id": "GO:0140293",
  "gene_symbol": "MACROD1",
  "gene_name": "ADP-ribose glycohydrolase MACROD1"
}